{
  "term_id": "GO:0005737",
  "gene_name": "Kelch-like protein 17",
  "gene": "UniProtKB:Q6TDP4",
  "gene_symbol": "KLHL17",
  "term_label": "cytoplasm"
}